apoptosome assembly [GO:0097314] (biological process) Sources: GOC:mtg_apoptosis Definition: The aggregation, arrangement and bonding together of the apoptosome, a multisubunit protein complex involved in the signaling phase of the apoptotic process. Relationships: is a type of protein-containing complex assembly [GO:0065003]; is part of GO:0097190 Regulation: regulated by GO:1905100; RO_0002212 by negative regulation of apoptosome assembly [GO:1905101]; positively regulated by positive regulation of apoptosome assembly [GO:1905102] Also known as: apoptosome formation